{
  "gene_name": "Neurexin-3",
  "gene": "UniProtKB:Q9Y4C0",
  "term_label": "adult behavior",
  "term_id": "GO:0030534",
  "gene_symbol": "NRXN3"
}